macula densa development [GO:0072024] (biological process) Relationships: is a type of nephron epithelium development [GO:0072009]; is part of juxtaglomerular apparatus development [GO:0072051] Definition: The process whose specific outcome is the progression of the macula densa over time, from its formation to the mature structure. The macula densa is an area of specialized cells in the distal tubule that makes contact with the vascular pole of the glomerulus. Subtypes: mesonephric macula densa development [GO:0061220], metanephric macula densa development [GO:0072227] Sources: GOC:mtg_kidney_jan10